{
  "gene_name": "Cytosolic carboxypeptidase 1",
  "gene": "UniProtKB:Q9UPW5",
  "gene_symbol": "AGTPBP1",
  "term_id": "UNKNOWN:0002",
  "term_label": "Unknown biological process"
}